{
  "gene_symbol": "DCTN2",
  "term_label": "centrosome",
  "gene": "UniProtKB:Q13561",
  "gene_name": "Dynactin subunit 2",
  "term_id": "GO:0005813"
}